{
  "gene_symbol": "ALX1",
  "term_label": "nucleus",
  "gene_name": "ALX homeobox protein 1",
  "term_id": "GO:0005634",
  "gene": "UniProtKB:Q15699"
}